{
  "gene_name": "Mitochondrial fission regulator 2",
  "gene_symbol": "MTFR2",
  "gene": "UniProtKB:Q6P444",
  "term_label": "aerobic respiration",
  "term_id": "GO:0009060"
}